tropomyosin binding [GO:0005523] (molecular function) Relationships: is a type of cytoskeletal protein binding [GO:0008092] Sources: GOC:curators, ISBN:0815316194 Definition: Binding to tropomyosin, a protein associated with actin filaments both in cytoplasm and, in association with troponin, in the thin filament of striated muscle.